{
  "gene": "UniProtKB:Q99519",
  "term_label": "ganglioside catabolic process",
  "gene_symbol": "NEU1",
  "gene_name": "Sialidase-1",
  "term_id": "GO:0006689"
}